{
  "term_id": "GO:0061631",
  "gene_symbol": "UBE2K",
  "gene_name": "Ubiquitin-conjugating enzyme E2 K",
  "gene": "UniProtKB:P61086",
  "term_label": "ubiquitin conjugating enzyme activity"
}